kynurenine 7,8-hydroxylase activity [GO:0050016] (molecular function) Also known as: kynurenate 7,8-hydroxylase activity, kynurenate,hydrogen-donor:oxygen oxidoreductase (hydroxylating), kynurenic acid hydroxylase activity, kynurenic hydroxylase activity Relationships: is a type of monooxygenase activity [GO:0004497]; is a type of GO:0016705 Sources: EC:1.14.99.2 Definition: Catalysis of the reaction: kynurenate + donor-H2 + O2 = 7,8-dihydro-7,8-dihydroxykynurenate + acceptor.